{
  "term_id": "GO:0031492",
  "gene": "UniProtKB:P60008",
  "gene_name": "Putative spermatid-specific linker histone H1-like protein",
  "gene_symbol": "H1-9P",
  "term_label": "nucleosomal DNA binding"
}